{
  "gene": "UniProtKB:Q9UQM7",
  "gene_name": "Calcium_calmodulin-dependent protein kinase type II subunit alpha",
  "term_id": "GO:1903076",
  "term_label": "regulation of protein localization to plasma membrane",
  "gene_symbol": "CAMK2A"
}